{
  "gene_symbol": "SLC5A5",
  "term_label": "Unknown cellular component",
  "gene_name": "Sodium_iodide cotransporter",
  "gene": "UniProtKB:Q92911",
  "term_id": "UNKNOWN:0003"
}